{
  "term_label": "endoplasmic reticulum membrane",
  "term_id": "GO:0005789",
  "gene_name": "Protein Aster-B",
  "gene_symbol": "GRAMD1B",
  "gene": "UniProtKB:Q3KR37"
}